{
  "term_label": "nucleus",
  "gene": "UniProtKB:P0C1H6",
  "term_id": "GO:0005634",
  "gene_name": "Histone H2B type F-M",
  "gene_symbol": "H2BW2"
}